{
  "term_label": "transcription elongation by RNA polymerase II",
  "term_id": "GO:0006368",
  "gene": "UniProtKB:Q96CJ1",
  "gene_name": "ELL-associated factor 2",
  "gene_symbol": "EAF2"
}